N-(4-aminobenzoyl)-L-glutamate synthetase activity [GO:0052625] (molecular function) References: PMID:19189963 Sources: MetaCyc:RXN-10884 Also known as: 4-aminobenzoate amino acid synthetase activity, 4-aminobenzoyl amino acid synthetase activity, p-aminobenzoate amino acid synthetase activity, p-aminobenzoyl amino acid synthetase activity, pABA amino acid synthetase activity Relationships: is a type of acid-amino acid ligase activity [GO:0016881] Definition: Catalysis of the reaction: 4-aminobenzoate + L-glutamate + ATP = N-(4-aminobenzoyl)-L-glutamate + AMP + diphosphate + H+.